{
  "term_id": "UNKNOWN:0001",
  "gene_symbol": "ZNF706",
  "gene": "UniProtKB:Q9Y5V0",
  "gene_name": "Zinc finger protein 706",
  "term_label": "Unknown molecular function"
}